{
  "gene_name": "L-serine dehydratase_L-threonine deaminase",
  "gene": "UniProtKB:P20132",
  "term_id": "UNKNOWN:0003",
  "gene_symbol": "SDS",
  "term_label": "Unknown cellular component"
}